{
  "term_id": "UNKNOWN:0003",
  "gene": "UniProtKB:P12980",
  "gene_symbol": "LYL1",
  "term_label": "Unknown cellular component",
  "gene_name": "Protein lyl-1"
}